{
  "gene": "UniProtKB:Q86UZ6",
  "term_id": "GO:0000122",
  "term_label": "negative regulation of transcription by RNA polymerase II",
  "gene_symbol": "ZBTB46",
  "gene_name": "Zinc finger and BTB domain-containing protein 46"
}